cuticle development [GO:0042335] (biological process) Definition: The chemical reactions and pathways resulting in the formation of a cuticle, the outer layer of some animals and plants, which acts to prevent water loss. Sources: ISBN:0192800825 Also known as: cuticle anabolism, cuticle biosynthesis, cuticle biosynthetic process, cuticle formation, cuticle synthesis Relationships: is_a anatomical structure development [GO:0048856]; is part of multicellular organism development [GO:0007275] Subtypes: GO:0040002, GO:0040003